{
  "term_label": "RNA polymerase II cis-regulatory region sequence-specific DNA binding",
  "gene": "UniProtKB:Q6ZMS4",
  "gene_symbol": "ZNF852",
  "gene_name": "Zinc finger protein 852",
  "term_id": "GO:0000978"
}